{
  "gene": "UniProtKB:Q969R5",
  "gene_name": "Lethal(3)malignant brain tumor-like protein 2",
  "gene_symbol": "L3MBTL2",
  "term_label": "chromatin binding",
  "term_id": "GO:0003682"
}